mast cell degranulation [GO:0043303] (biological process) Regulation: regulated by GO:0043304; negatively regulated by GO:0043305; positively regulated by positive regulation of mast cell degranulation [GO:0043306] Sources: ISBN:0781735149 Definition: The regulated exocytosis of secretory granules containing preformed mediators such as histamine, serotonin, and neutral proteases by a mast cell. Also known as: mast cell granule exocytosis Relationships: is a type of lysosome localization [GO:0032418]; is a type of leukocyte degranulation [GO:0043299]; is a type of GO:0051656; is part of mast cell activation involved in immune response [GO:0002279]; is part of mast cell mediated immunity [GO:0002448]